{
  "term_label": "Unknown molecular function",
  "term_id": "UNKNOWN:0001",
  "gene": "UniProtKB:Q3MIV0",
  "gene_symbol": "KRTAP22-1",
  "gene_name": "Keratin-associated protein 22-1"
}